{
  "gene_symbol": "FN1",
  "gene": "UniProtKB:P02751",
  "term_label": "cell-matrix adhesion",
  "term_id": "GO:0007160",
  "gene_name": "Fibronectin"
}